negative regulation of hypersensitivity [GO:0002884] (biological process) Sources: GOC:add Also known as: down regulation of hypersensitivity, down-regulation of hypersensitivity, downregulation of hypersensitivity, inhibition of hypersensitivity Relationships: is a type of negative regulation of acute inflammatory response to antigenic stimulus [GO:0002865]; is a type of regulation of hypersensitivity [GO:0002883]; negatively regulates GO:0002524 Definition: Any process that stops, prevents, or reduces the frequency, rate, or extent of hypersensitivity. Subtypes: negative regulation of type III hypersensitivity [GO:0001804], GO:0001808, negative regulation of type I hypersensitivity [GO:0001811], GO:0002893